{
  "gene": "UniProtKB:A0A075B6J1",
  "term_id": "GO:0006955",
  "gene_name": "Immunoglobulin lambda variable 5-37",
  "term_label": "immune response",
  "gene_symbol": "IGLV5-37"
}